{
  "term_id": "GO:0007165",
  "gene_symbol": "PLPPR3",
  "gene": "UniProtKB:Q6T4P5",
  "gene_name": "Phospholipid phosphatase-related protein type 3",
  "term_label": "signal transduction"
}